negative regulation of protein localization to plasma membrane [GO:1903077] (biological process) References: PMID:11602640 Sources: GOC:BHF, GOC:TermGenie, GOC:rl, GO_REF:0000058 Relationships: is a type of regulation of protein localization to plasma membrane [GO:1903076]; is a type of negative regulation of protein localization to cell periphery [GO:1904376]; is a type of negative regulation of protein localization to membrane [GO:1905476]; negatively regulates protein localization to plasma membrane [GO:0072659] Subtypes: negative regulation of Golgi to plasma membrane protein transport [GO:0042997], negative regulation of protein localization to medial cortex [GO:0140325], negative regulation of endosome to plasma membrane protein transport [GO:1905750] Also known as: down regulation of protein localisation in plasma membrane, down regulation of protein localization in plasma membrane, down regulation of protein localization to plasma membrane, down-regulation of protein localisation in plasma membrane, down-regulation of protein localization in plasma membrane, down-regulation of protein localization to plasma membrane, downregulation of protein localisation in plasma membrane, downregulation of protein localization in plasma membrane, downregulation of protein localization to plasma membrane, negative regulation of protein localization in plasma membrane, inhibition of protein localisation in plasma membrane, inhibition of protein localization in plasma membrane, inhibition of protein localization to plasma membrane, inhibition of protein targeting to plasma membrane, inhibition of protein-plasma membrane targeting, down regulation of protein targeting to plasma membrane, down regulation of protein-plasma membrane targeting, down-regulation of protein targeting to plasma membrane, down-regulation of protein-plasma membrane targeting, downregulation of protein targeting to plasma membrane, downregulation of protein-plasma membrane targeting, negative regulation of establishment of protein localisation in plasma membrane, negative regulation of establishment of protein localization in plasma membrane, negative regulation of establishment of protein localization to plasma membrane, negative regulation of protein localisation in plasma membrane, negative regulation of protein targeting to plasma membrane, negative regulation of protein-plasma membrane targeting Definition: Any process that stops, prevents or reduces the frequency, rate or extent of protein localization to plasma membrane.